symbiont-mediated perturbation of host cell cycle G0/G1 transition checkpoint [GO:0039646] (BP) Relationships: is a type of symbiont-mediated perturbation of host cellular process [GO:0044068] Also known as: G0/G1 host cell cycle checkpoint dysregulation by virus, modulation by virus of host G0/G1 transition checkpoint, perturbation by virus of host G0/G1 transition checkpoint Sources: VZ:880 Definition: A process in which a symbiont interferes with the normal execution of the host cell G0/G1 transition checkpoint. The host is defined as the larger of the organisms involved in a symbiotic interaction. Some viruses benefit from keeping cells in resting state (G0), while others favor entry through G1 and subsequent cell division to replicate more efficiently.